corticotropin-releasing hormone secretion [GO:0043396] (biological process) Relationships: is a type of GO:0030072 Definition: The regulated release of corticotropin-releasing hormone (CRH), a polypeptide hormone involved in the stress response. CRH is produced by the hypothalamus and stimulates corticotropic cells of the anterior lobe of the pituitary to produce corticotropic hormone (CTH) and other biologically active substances e.g. 2-endorphin, release of CRH is affected by serum levels of cortisol, by stress and by the sleep/wake cycle. Regulation: regulated by GO:0043397; negatively regulated by negative regulation of corticotropin-releasing hormone secretion [GO:0051465]; positively regulated by positive regulation of corticotropin-releasing hormone secretion [GO:0051466] References: PMID:11027914 Sources: GOC:go_curators Also known as: CRF secretion, CRH secretion, corticotropin-releasing factor secretion